{
  "term_id": "GO:0008093",
  "gene": "UniProtKB:Q12955",
  "gene_symbol": "ANK3",
  "gene_name": "Ankyrin-3",
  "term_label": "cytoskeletal anchor activity"
}